{
  "term_id": "GO:0090435",
  "gene_name": "Lamin-B1",
  "term_label": "protein localization to nuclear envelope",
  "gene_symbol": "LMNB1",
  "gene": "UniProtKB:P20700"
}